{
  "gene": "UniProtKB:Q9Y224",
  "term_label": "RNA binding",
  "gene_symbol": "RTRAF",
  "gene_name": "RNA transcription, translation and transport factor protein",
  "term_id": "GO:0003723"
}